regulation of dendrite morphogenesis [GO:0048814] (biological process) Definition: Any process that modulates the frequency, rate or extent of dendrite morphogenesis. Subtypes: negative regulation of dendrite morphogenesis [GO:0050774], positive regulation of dendrite morphogenesis [GO:0050775] Relationships: is a type of GO:0022603; is a type of regulation of dendrite development [GO:0050773]; regulates GO:0048813 Sources: GOC:ai